{
  "term_label": "SUMO transferase activity",
  "term_id": "GO:0019789",
  "gene_name": "RanBP2-like and GRIP domain-containing protein 4",
  "gene": "UniProtKB:Q7Z3J3",
  "gene_symbol": "RGPD4"
}